{
  "gene": "UniProtKB:P01574",
  "term_label": "adaptive immune response",
  "gene_symbol": "IFNB1",
  "gene_name": "Interferon beta",
  "term_id": "GO:0002250"
}